respiratory chemosensitivity [GO:0160061] (biological process) References: PMID:26068853 Definition: A homeostatic process by which the sensing of CO2 and/or H+ by the brain leads to appropriate altering in breathing to regulate blood gas and tissue pH. Relationships: is_a multicellular organismal-level homeostasis [GO:0048871]